virus maturation [GO:0019075] (biological process) Also known as: viral maturation, bacteriophage maturation Relationships: is a type of viral process [GO:0016032]; is part of GO:0019058 Sources: ISBN:0781718325 Definition: The refolding and structural rearrangements of virion parts to transition from the intermediate virion to the more mature virion. Maturation usually involves proteolysis events and changes in the folding of the virion proteins. Can occur inside the host cell or after release.